{
  "term_id": "GO:0000422",
  "term_label": "autophagy of mitochondrion",
  "gene_name": "Serine_threonine-protein kinase PINK1, mitochondrial",
  "gene": "UniProtKB:Q9BXM7",
  "gene_symbol": "PINK1"
}